{
  "gene_name": "Heat shock transcription factor, X-linked",
  "term_id": "GO:0005634",
  "gene_symbol": "HSFX2",
  "term_label": "nucleus",
  "gene": "UniProtKB:Q9UBD0"
}